{
  "gene_name": "Ribosomal RNA processing protein 1 homolog A",
  "term_label": "transcription coactivator activity",
  "gene": "UniProtKB:P56182",
  "term_id": "GO:0003713",
  "gene_symbol": "RRP1"
}